{
  "term_label": "ubiquitin-dependent protein catabolic process",
  "gene_name": "E3 ubiquitin-protein ligase RNF6",
  "term_id": "GO:0006511",
  "gene": "UniProtKB:Q9Y252",
  "gene_symbol": "RNF6"
}